{
  "gene_name": "Kinesin-like protein KIF1B",
  "gene_symbol": "KIF1B",
  "term_label": "ATP hydrolysis activity",
  "term_id": "GO:0016887",
  "gene": "UniProtKB:O60333"
}